{
  "gene_symbol": "RRP7BP",
  "gene_name": "Putative ribosomal RNA-processing protein 7 homolog B",
  "gene": "UniProtKB:Q9NSQ0",
  "term_id": "GO:0000028",
  "term_label": "ribosomal small subunit assembly"
}